mitochondrial proton-transporting ATP synthase complex assembly [GO:0033615] (biological process) Definition: The aggregation, arrangement and bonding together of a proton-transporting ATP synthase in the mitochondrial inner membrane. Relationships: is a type of mitochondrial respiratory chain complex assembly [GO:0033108]; is a type of proton-transporting ATP synthase complex assembly [GO:0043461] Sources: GOC:mah